{
  "gene": "UniProtKB:P08686",
  "term_label": "glucocorticoid biosynthetic process",
  "gene_symbol": "CYP21A2",
  "gene_name": "Steroid 21-hydroxylase",
  "term_id": "GO:0006704"
}